{
  "gene_name": "Ras-related protein Rab-12",
  "gene": "UniProtKB:Q6IQ22",
  "gene_symbol": "RAB12",
  "term_id": "GO:0032456",
  "term_label": "endocytic recycling"
}